regulation of interleukin-1 beta production [GO:0032651] (BP) Sources: GOC:mah Relationships: is a type of regulation of interleukin-1 production [GO:0032652]; regulates GO:0032611 Definition: Any process that modulates the frequency, rate, or extent of interleukin-1 beta production. Also known as: regulation of IL-1 beta production, regulation of interleukin-1 beta biosynthetic process, regulation of interleukin-1 beta secretion Subtypes: negative regulation of interleukin-1 beta production [GO:0032691], GO:0032731